{
  "term_label": "nucleus",
  "gene_symbol": "SIRT6",
  "gene": "UniProtKB:Q8N6T7",
  "term_id": "GO:0005634",
  "gene_name": "NAD-dependent protein deacylase sirtuin-6"
}